{
  "term_label": "positive regulation of B cell receptor signaling pathway",
  "gene_symbol": "STAP1",
  "gene_name": "Signal-transducing adaptor protein 1",
  "term_id": "GO:0050861",
  "gene": "UniProtKB:Q9ULZ2"
}